{
  "gene_name": "Xylosyltransferase 2",
  "term_id": "GO:0030158",
  "term_label": "protein xylosyltransferase activity",
  "gene": "UniProtKB:Q9H1B5",
  "gene_symbol": "XYLT2"
}